{
  "term_id": "GO:0061629",
  "term_label": "RNA polymerase II-specific DNA-binding transcription factor binding",
  "gene_symbol": "ANKRD2",
  "gene": "UniProtKB:Q9GZV1",
  "gene_name": "Ankyrin repeat domain-containing protein 2"
}